{
  "gene": "UniProtKB:P62310",
  "term_label": "P-body assembly",
  "term_id": "GO:0033962",
  "gene_name": "U6 snRNA-associated Sm-like protein LSm3",
  "gene_symbol": "LSM3"
}